{
  "term_id": "GO:0000978",
  "term_label": "RNA polymerase II cis-regulatory region sequence-specific DNA binding",
  "gene": "UniProtKB:Q9ULD5",
  "gene_name": "Zinc finger protein 777",
  "gene_symbol": "ZNF777"
}